{
  "gene": "UniProtKB:Q8IY81",
  "gene_symbol": "FTSJ3",
  "gene_name": "pre-rRNA 2'-O-ribose RNA methyltransferase FTSJ3",
  "term_label": "preribosome, large subunit precursor",
  "term_id": "GO:0030687"
}